{
  "gene_name": "Ras association domain-containing protein 8",
  "gene": "UniProtKB:Q8NHQ8",
  "term_label": "Unknown molecular function",
  "gene_symbol": "RASSF8",
  "term_id": "UNKNOWN:0001"
}